{
  "term_label": "nuclear pore",
  "term_id": "GO:0005643",
  "gene_name": "RANBP2-like and GRIP domain-containing protein 1",
  "gene": "UniProtKB:P0DJD0",
  "gene_symbol": "RGPD1"
}